{
  "term_label": "chloride channel activity",
  "gene_name": "Bestrophin-2",
  "gene": "UniProtKB:Q8NFU1",
  "gene_symbol": "BEST2",
  "term_id": "GO:0005254"
}